{
  "term_id": "GO:0005634",
  "gene_symbol": "DLX5",
  "term_label": "nucleus",
  "gene_name": "Homeobox protein DLX-5",
  "gene": "UniProtKB:P56178"
}